ethanol-acetate fermentation to butyrate and caproate [GO:0019672] (biological process) Sources: MetaCyc:P127-PWY Relationships: is_a non-glycolytic fermentation [GO:0019662] Definition: The anaerobic chemical reactions and pathways resulting in the breakdown of ethanol and acetate to butyrate and caproate, yielding energy in the form of ATP.